establishment of protein localization to mitochondrial membrane involved in mitochondrial fission [GO:0090152] (biological process) Also known as: establishment of protein localisation in mitochondrial membrane involved in mitochondrial fission, establishment of protein localization in mitochondrial membrane involved in mitochondrial fission Sources: GOC:ascb_2009, GOC:dph, GOC:tb Relationships: is a type of GO:0090151; is part of GO:0000266 Definition: The directed movement of a protein to a specific location in the mitochondrial membrane that contributes to mitochondrial fission.